{
  "gene_name": "Forkhead box protein L1",
  "gene": "UniProtKB:Q12952",
  "gene_symbol": "FOXL1",
  "term_label": "DNA-binding transcription factor activity, RNA polymerase II-specific",
  "term_id": "GO:0000981"
}